epithelial cell proliferation involved in lung morphogenesis [GO:0060502] (biological process) Definition: The multiplication or reproduction of epithelial cells, resulting in the expansion of a cell population that contributes to the shaping of the lung. Subtypes: epithelial cell proliferation involved in lung bud dilation [GO:0060505] Regulation: positively regulated by GO:0060501; regulated by regulation of epithelial cell proliferation involved in lung morphogenesis [GO:2000794]; negatively regulated by negative regulation of epithelial cell proliferation involved in lung morphogenesis [GO:2000795] Relationships: is_a epithelial cell proliferation [GO:0050673]; is part of lung morphogenesis [GO:0060425]; is part of lung epithelium development [GO:0060428] Sources: GOC:dph